positive regulation of vascular associated smooth muscle cell differentiation involved in phenotypic switching [GO:1905932] (biological process) Relationships: is a type of positive regulation of vascular associated smooth muscle cell differentiation [GO:1905065]; is_a positive regulation of cell differentiation involved in phenotypic switching [GO:1905917]; is a type of regulation of vascular associated smooth muscle cell differentiation involved in phenotypic switching [GO:1905930]; positively regulates vascular associated smooth muscle cell differentiation involved in phenotypic switching [GO:1905420] References: PMID:25089138 Sources: GOC:BHF, GOC:BHF_miRNA, GOC:TermGenie, GOC:rph, GO_REF:0000058 Definition: Any process that activates or increases the frequency, rate or extent of vascular smooth muscle cell differentiation involved in phenotypic switching. Also known as: positive regulation of VSMC differentiation involved in phenotypic switching, positive regulation of vascular smooth muscle cell differentiation involved in phenotypic switching, up regulation of VSMC differentiation involved in phenotypic switching, up regulation of vascular associated smooth muscle cell differentiation involved in phenotypic switching, up regulation of vascular smooth muscle cell differentiation involved in phenotypic switching, up-regulation of VSMC differentiation involved in phenotypic switching, up-regulation of vascular associated smooth muscle cell differentiation involved in phenotypic switching, up-regulation of vascular smooth muscle cell differentiation involved in phenotypic switching, upregulation of VSMC differentiation involved in phenotypic switching, upregulation of vascular associated smooth muscle cell differentiation involved in phenotypic switching, upregulation of vascular smooth muscle cell differentiation involved in phenotypic switching, activation of VSMC differentiation involved in phenotypic switching, activation of vascular associated smooth muscle cell differentiation involved in phenotypic switching, activation of vascular smooth muscle cell differentiation involved in phenotypic switching, activation of VSMC differentiation involved in phenotypic dimorphism, activation of vascular associated smooth muscle cell differentiation involved in phenotypic dimorphism, activation of vascular smooth muscle cell differentiation involved in phenotypic dimorphism, positive regulation of VSMC differentiation involved in phenotypic dimorphism, positive regulation of vascular associated smooth muscle cell differentiation involved in phenotypic dimorphism, positive regulation of vascular smooth muscle cell differentiation involved in phenotypic dimorphism, up regulation of VSMC differentiation involved in phenotypic dimorphism, up regulation of vascular associated smooth muscle cell differentiation involved in phenotypic dimorphism, up regulation of vascular smooth muscle cell differentiation involved in phenotypic dimorphism, up-regulation of VSMC differentiation involved in phenotypic dimorphism, up-regulation of vascular associated smooth muscle cell differentiation involved in phenotypic dimorphism, up-regulation of vascular smooth muscle cell differentiation involved in phenotypic dimorphism, upregulation of VSMC differentiation involved in phenotypic dimorphism, upregulation of vascular associated smooth muscle cell differentiation involved in phenotypic dimorphism, upregulation of vascular smooth muscle cell differentiation involved in phenotypic dimorphism